heptose-1-phosphate adenylyltransferase activity [GO:0033786] (MF) Sources: MetaCyc:RXN0-4342 Relationships: is a type of adenylyltransferase activity [GO:0070566] Definition: Catalysis of the reaction: D-beta-D-heptose-1-phosphate + ATP = ADP-D-glycero-D-manno-heptose. Also known as: D-beta-D-heptose 1-phosphate adenylyltransferase activity, heptose 1-phosphate adenyltransferase activity